{
  "term_id": "GO:0051123",
  "gene_name": "TATA-box-binding protein-associated factor 11-like protein 8",
  "gene": "UniProtKB:P0DW13",
  "term_label": "RNA polymerase II preinitiation complex assembly",
  "gene_symbol": "TAF11L8"
}